{
  "gene": "UniProtKB:O14514",
  "gene_name": "Adhesion G protein-coupled receptor B1",
  "term_label": "dendrite",
  "gene_symbol": "ADGRB1",
  "term_id": "GO:0030425"
}